{
  "term_label": "T cell receptor signaling pathway",
  "gene_symbol": "CLEC2D",
  "gene": "UniProtKB:Q9UHP7",
  "term_id": "GO:0050852",
  "gene_name": "C-type lectin domain family 2 member D"
}